P granule disassembly [GO:1903864] (biological process) Also known as: germline granule disassembly, polar granule disassembly References: PMID:25535836 Sources: GOC:TermGenie, GOC:kmv, GO_REF:0000079 Relationships: is a type of GO:0030719; is a type of organelle disassembly [GO:1903008] Definition: The disaggregation of a P granule into its constituent components.